tendon development [GO:0035989] (biological process) Definition: The process whose specific outcome is the progression of a tendon over time, from its formation to the mature structure. A tendon is a fibrous, strong, connective tissue that connects muscle to bone or integument and is capable of withstanding tension. Tendons and muscles work together to exert a pulling force. Relationships: is a type of connective tissue development [GO:0061448] Also known as: sinew development References: PMID:21412429 Sources: GOC:yaf, UBERON:0000043